negative regulation of voltage-gated calcium channel activity [GO:1901386] (biological process) Definition: Any process that stops, prevents or reduces the frequency, rate or extent of voltage-gated calcium channel activity. Sources: GOC:BHF, GOC:TermGenie Also known as: down regulation of depolarization-activated calcium channel, down-regulation of depolarization-activated calcium channel, downregulation of depolarization-activated calcium channel, inhibition of depolarization-activated calcium channel, negative regulation of depolarization-activated calcium channel, down regulation of depolarization-activated voltage gated calcium channel activity, down regulation of depolarization-activated voltage-gated calcium channel, down regulation of depolarization-activated voltage-gated calcium channel activity, down regulation of voltage gated calcium channel activity, down regulation of voltage-dependent calcium channel activity, down regulation of voltage-gated calcium channel activity, down regulation of voltage-gated calcium ion channel activity, down regulation of voltage-sensitive calcium channel, down-regulation of depolarization-activated voltage gated calcium channel activity, down-regulation of depolarization-activated voltage-gated calcium channel, down-regulation of depolarization-activated voltage-gated calcium channel activity, down-regulation of voltage gated calcium channel activity, down-regulation of voltage-dependent calcium channel activity, down-regulation of voltage-gated calcium channel activity, down-regulation of voltage-gated calcium ion channel activity, down-regulation of voltage-sensitive calcium channel, downregulation of depolarization-activated voltage gated calcium channel activity, downregulation of depolarization-activated voltage-gated calcium channel, downregulation of depolarization-activated voltage-gated calcium channel activity, downregulation of voltage gated calcium channel activity, downregulation of voltage-dependent calcium channel activity, downregulation of voltage-gated calcium channel activity, downregulation of voltage-gated calcium ion channel activity, downregulation of voltage-sensitive calcium channel, inhibition of depolarization-activated voltage gated calcium channel activity, inhibition of depolarization-activated voltage-gated calcium channel, inhibition of depolarization-activated voltage-gated calcium channel activity, inhibition of voltage gated calcium channel activity, inhibition of voltage-dependent calcium channel activity, inhibition of voltage-gated calcium ion channel activity, inhibition of voltage-sensitive calcium channel, negative regulation of depolarization-activated voltage gated calcium channel activity, negative regulation of depolarization-activated voltage-gated calcium channel, negative regulation of depolarization-activated voltage-gated calcium channel activity, negative regulation of voltage gated calcium channel activity, negative regulation of voltage-dependent calcium channel activity, negative regulation of voltage-gated calcium ion channel activity, negative regulation of voltage-sensitive calcium channel, down regulation of dihydropyridine-sensitive calcium channel activity, down-regulation of dihydropyridine-sensitive calcium channel activity, downregulation of dihydropyridine-sensitive calcium channel activity, inhibition of dihydropyridine-sensitive calcium channel activity, inhibition of voltage-gated calcium channel activity, negative regulation of dihydropyridine-sensitive calcium channel activity Relationships: is a type of negative regulation of calcium ion transmembrane transporter activity [GO:1901020]; is a type of GO:1901385; RO_0002212 voltage-gated calcium channel activity [GO:0005245] Subtypes: GO:1901842